{
  "term_label": "double-stranded RNA binding",
  "gene": "UniProtKB:Q8NCV1",
  "gene_name": "Adenosine deaminase domain-containing protein 2",
  "term_id": "GO:0003725",
  "gene_symbol": "ADAD2"
}